{
  "gene": "UniProtKB:Q96RK0",
  "term_label": "DNA-binding transcription factor activity, RNA polymerase II-specific",
  "gene_symbol": "CIC",
  "term_id": "GO:0000981",
  "gene_name": "Protein capicua homolog"
}